{
  "gene_symbol": "IRX5",
  "gene_name": "Iroquois-class homeodomain protein IRX-5",
  "gene": "UniProtKB:P78411",
  "term_id": "GO:0030182",
  "term_label": "neuron differentiation"
}